one-carbon compound transport [GO:0019755] (biological process) Subtypes: carbon dioxide transport [GO:0015670], cyanate transport [GO:0015704], urea transport [GO:0015840], GO:0015843 Also known as: one carbon compound transport Sources: GOC:ai Definition: The directed movement of one-carbon compounds into, out of or within a cell, or between cells, by means of some agent such as a transporter or pore. Relationships: is a type of transport [GO:0006810]